{
  "term_label": "hormone activity",
  "gene_symbol": "A0A2R8Y747",
  "gene": "UniProtKB:A0A2R8Y747",
  "gene_name": "Uncharacterized protein",
  "term_id": "GO:0005179"
}